{
  "gene_symbol": "SCLY",
  "gene_name": "Selenocysteine lyase",
  "term_id": "UNKNOWN:0001",
  "term_label": "Unknown molecular function",
  "gene": "UniProtKB:Q96I15"
}